{
  "gene": "UniProtKB:Q9HAE3",
  "gene_symbol": "CLXN",
  "term_id": "UNKNOWN:0003",
  "gene_name": "Calaxin",
  "term_label": "Unknown cellular component"
}